{
  "gene": "UniProtKB:Q14457",
  "gene_name": "Beclin-1",
  "gene_symbol": "BECN1",
  "term_id": "GO:0000045",
  "term_label": "autophagosome assembly"
}